{
  "gene_name": "Transcription factor Sp1",
  "gene_symbol": "SP1",
  "gene": "UniProtKB:P08047",
  "term_id": "GO:0005634",
  "term_label": "nucleus"
}